protein localization to old growing cell tip [GO:1903858] (biological process) Relationships: is_a protein localization to growing cell tip [GO:1902486] Definition: A process in which a protein is transported to, or maintained in, a location within an old growing cell tip. Also known as: protein localisation in old growing cell tip, protein localisation to old growing cell tip, protein localization in old growing cell tip References: PMID:17895368 Sources: GOC:TermGenie, GO_REF:0000087